{
  "term_id": "GO:0007423",
  "gene_name": "Paired box protein Pax-2",
  "gene_symbol": "PAX2",
  "gene": "UniProtKB:Q02962",
  "term_label": "sensory organ development"
}